{
  "gene_symbol": "TMED1",
  "term_label": "intracellular protein transport",
  "gene": "UniProtKB:Q13445",
  "term_id": "GO:0006886",
  "gene_name": "Transmembrane emp24 domain-containing protein 1"
}